{
  "gene_name": "Centromere protein J",
  "gene": "UniProtKB:Q9HC77",
  "term_label": "tubulin binding",
  "term_id": "GO:0015631",
  "gene_symbol": "CENPJ"
}